regulation of phenotypic switching [GO:1900239] (biological process) Definition: Any process that modulates the frequency, rate or extent of phenotypic switching. Subtypes: negative regulation of phenotypic switching [GO:1900240], GO:1900241 Relationships: is a type of regulation of cellular process [GO:0050794]; regulates GO:0036166 Also known as: regulation of phenotypic dimorphism Sources: GOC:TermGenie, GOC:di